S-layer organization [GO:0045232] (biological process) Sources: GOC:ai Also known as: S-layer organisation, S-layer organization and biogenesis Definition: A process that is carried out at the cellular level which results in the assembly, arrangement of constituent parts, or disassembly of an S-layer enveloping the cell. The S-layer is a crystalline protein layer surrounding some bacteria. Relationships: is a type of external encapsulating structure organization [GO:0045229]